mitotic actomyosin contractile ring assembly [GO:1903475] (biological process) Relationships: is a type of actomyosin contractile ring assembly [GO:0000915]; is a type of assembly of actomyosin apparatus involved in mitotic cytokinesis [GO:1902407] Sources: GOC:TermGenie, GOC:mtg_cell_cycle, GO_REF:0000060 Definition: Any actomyosin contractile ring assembly that is involved in mitotic cytokinesis. Regulation: regulated by regulation of mitotic actomyosin contractile ring assembly [GO:1903499]; negatively regulated by negative regulation of mitotic actomyosin contractile ring assembly [GO:1903500]; positively regulated by positive regulation of mitotic actomyosin contractile ring assembly [GO:1903501] Also known as: actomyosin contractile ring assembly involved in cytokinesis after mitosis, contractile ring assembly involved in mitotic cytokinesis, cytokinesis, actomyosin contractile ring assembly involved in mitotic cytokinesis